{
  "gene_symbol": "AKT2",
  "term_id": "GO:0004674",
  "term_label": "protein serine/threonine kinase activity",
  "gene": "UniProtKB:P31751",
  "gene_name": "RAC-beta serine_threonine-protein kinase"
}